{
  "gene": "UniProtKB:P31644",
  "term_id": "GO:0004890",
  "term_label": "GABA-A receptor activity",
  "gene_symbol": "GABRA5",
  "gene_name": "Gamma-aminobutyric acid receptor subunit alpha-5"
}